{
  "gene_name": "Mediator of RNA polymerase II transcription subunit 12-like protein",
  "gene_symbol": "MED12L",
  "term_id": "GO:0003713",
  "gene": "UniProtKB:Q86YW9",
  "term_label": "transcription coactivator activity"
}